monodictyphenone biosynthetic process [GO:1900815] (biological process) Regulation: regulated by regulation of monodictyphenone biosynthetic process [GO:1900843]; negatively regulated by negative regulation of monodictyphenone biosynthetic process [GO:1900844]; positively regulated by positive regulation of monodictyphenone biosynthetic process [GO:1900845] Relationships: is a type of ketone biosynthetic process [GO:0042181]; is a type of GO:0044550; is_a phenol-containing compound biosynthetic process [GO:0046189]; is a type of carboxylic acid biosynthetic process [GO:0046394]; is a type of GO:1900813 Definition: The chemical reactions and pathways resulting in the formation of monodictyphenone. Also known as: monodictyphenone anabolism, monodictyphenone biosynthesis, monodictyphenone formation, monodictyphenone synthesis Sources: GOC:TermGenie, GOC:di